{
  "gene_symbol": "CSNK2A2",
  "term_label": "DNA damage response",
  "gene_name": "Casein kinase II subunit alpha'",
  "gene": "UniProtKB:P19784",
  "term_id": "GO:0006974"
}